{
  "term_label": "Golgi apparatus",
  "gene": "UniProtKB:Q4J6C6",
  "term_id": "GO:0005794",
  "gene_name": "Prolyl endopeptidase-like",
  "gene_symbol": "PREPL"
}